{
  "term_label": "positive regulation of transcription by RNA polymerase II",
  "gene_symbol": "PPARGC1A",
  "term_id": "GO:0045944",
  "gene_name": "Peroxisome proliferator-activated receptor gamma coactivator 1-alpha",
  "gene": "UniProtKB:Q9UBK2"
}